{
  "term_label": "small GTPase binding",
  "gene": "UniProtKB:A1L390",
  "gene_symbol": "PLEKHG3",
  "gene_name": "Pleckstrin homology domain-containing family G member 3",
  "term_id": "GO:0031267"
}